aminodeoxychorismate synthase complex [GO:0009356] (cellular component) Relationships: is a type of intracellular protein-containing complex [GO:0140535]; is a type of catalytic complex [GO:1902494] Also known as: ADC synthase complex, 4-amino-4-deoxychorismate synthase complex, p-aminobenzoate synthetase complex Definition: A heterodimeric protein complex that possesses 4-amino-4-deoxychorismate synthase activity. References: PMID:2251281, PMID:7592344